Golgi disassembly [GO:0090166] (biological process) Also known as: Golgi apparatus disassembly Definition: A cellular process that results in the breakdown of a Golgi apparatus that contributes to Golgi inheritance. Relationships: is a type of Golgi organization [GO:0007030]; is a type of organelle disassembly [GO:1903008]; BFO_0000050 Golgi inheritance [GO:0048313] Sources: GOC:ascb_2009, GOC:dph, GOC:tb